{
  "term_id": "GO:0046546",
  "gene_name": "Muellerian-inhibiting factor",
  "gene": "UniProtKB:P03971",
  "term_label": "development of primary male sexual characteristics",
  "gene_symbol": "AMH"
}